{
  "term_label": "neuron fate commitment",
  "gene": "UniProtKB:Q8N100",
  "gene_name": "Transcription factor ATOH7",
  "gene_symbol": "ATOH7",
  "term_id": "GO:0048663"
}